 [go#goslim:drosophila] Note: Drosophila GO slim